regulation of branchiomeric skeletal muscle development [GO:0014711] (biological process) Definition: Any process that modulates the frequency, rate or extent of branchiomeric skeletal muscle development. Branchiomeric skeletal muscle development is the process whose specific outcome is the progression of the branchiomeric skeletal muscle over time, from its formation to the mature structure. Sources: GOC:mtg_muscle Subtypes: positive regulation of branchiomeric skeletal muscle development [GO:0014712], GO:0014713 Relationships: is a type of regulation of skeletal muscle tissue development [GO:0048641]; regulates branchiomeric skeletal muscle development [GO:0014707]